{
  "term_id": "GO:0060048",
  "gene": "UniProtKB:P09493",
  "term_label": "cardiac muscle contraction",
  "gene_name": "Tropomyosin alpha-1 chain",
  "gene_symbol": "TPM1"
}